{
  "gene_symbol": "PINK1",
  "term_id": "GO:0005739",
  "gene": "UniProtKB:Q9BXM7",
  "gene_name": "Serine_threonine-protein kinase PINK1, mitochondrial",
  "term_label": "mitochondrion"
}